vitellogenin receptor activity [GO:0008196] (molecular function) Relationships: is a type of GO:0038024 Definition: Receiving vitellogenin, and delivering vitellogenin into the cell via endocytosis. References: PMID:12429745 Sources: GOC:bf